{
  "term_id": "GO:0004653",
  "term_label": "polypeptide N-acetylgalactosaminyltransferase activity",
  "gene_symbol": "GALNT13",
  "gene_name": "Polypeptide N-acetylgalactosaminyltransferase 13",
  "gene": "UniProtKB:Q8IUC8"
}